{
  "gene_name": "Apolipoprotein L6",
  "term_label": "Unknown biological process",
  "term_id": "UNKNOWN:0002",
  "gene_symbol": "APOL6",
  "gene": "UniProtKB:Q9BWW8"
}